NADH dehydrogenase complex assembly [GO:0010257] (biological process) Subtypes: NADH dehydrogenase complex (plastoquinone) assembly [GO:0010258], mitochondrial respiratory chain complex I assembly [GO:0032981] Relationships: is a type of protein-containing complex assembly [GO:0065003] Definition: The aggregation, arrangement and bonding together of a set of components to form an NADH dehydrogenase complex. Sources: GOC:sm